CoA-dependent peptidyl-lysine N6-palmitoyltransferase activity [GO:0140772] (molecular function) References: PMID:30061757 Relationships: is a type of GO:0018031 Definition: Catalysis of the reaction: L-lysyl-[protein] + hexadecanoyl-CoA = CoA + H+ + N(6)-hexadecanoyl-L-lysyl-[protein].